{
  "term_label": "chromatin",
  "gene": "UniProtKB:Q29RF7",
  "gene_symbol": "PDS5A",
  "term_id": "GO:0000785",
  "gene_name": "Sister chromatid cohesion protein PDS5 homolog A"
}